positive regulation of peptidyl-threonine phosphorylation [GO:0010800] (BP) Sources: GOC:dph, GOC:tb Definition: Any process that increases the frequency, rate or extent of peptidyl-threonine phosphorylation. Peptidyl-threonine phosphorylation is the phosphorylation of peptidyl-threonine to form peptidyl-O-phospho-L-threonine. Relationships: is a type of positive regulation of protein phosphorylation [GO:0001934]; is a type of GO:0010799; positively regulates peptidyl-threonine phosphorylation [GO:0018107]